lung goblet cell differentiation [GO:0060480] (biological process) Relationships: is a type of lung secretory cell differentiation [GO:0061140]; is part of GO:0060481 Definition: The process in which a relatively unspecialized cell acquires specialized features of a lung goblet cell. A goblet cell is a cell of the epithelial lining that produces and secretes mucins. Also known as: pulmonary goblet cell differentiation Sources: GOC:dph, GOC:mtg_lung Regulation: regulated by GO:1901249; negatively regulated by GO:1901250; positively regulated by positive regulation of lung goblet cell differentiation [GO:1901251]